{
  "gene_name": "Tectonic-3",
  "term_id": "GO:0060271",
  "term_label": "cilium assembly",
  "gene": "UniProtKB:Q6NUS6",
  "gene_symbol": "TCTN3"
}